{
  "gene_symbol": "ARL6",
  "term_label": "cytoplasm",
  "gene": "UniProtKB:Q9H0F7",
  "term_id": "GO:0005737",
  "gene_name": "ADP-ribosylation factor-like protein 6"
}